{
  "term_id": "GO:0000978",
  "term_label": "RNA polymerase II cis-regulatory region sequence-specific DNA binding",
  "gene": "UniProtKB:O75364",
  "gene_name": "Pituitary homeobox 3",
  "gene_symbol": "PITX3"
}